{
  "gene_symbol": "RNF113B",
  "term_id": "GO:0005684",
  "term_label": "U2-type spliceosomal complex",
  "gene_name": "RING finger protein 113B",
  "gene": "UniProtKB:Q8IZP6"
}